{
  "term_id": "GO:0001540",
  "term_label": "amyloid-beta binding",
  "gene_name": "Integrin beta-2",
  "gene": "UniProtKB:P05107",
  "gene_symbol": "ITGB2"
}